{
  "gene": "UniProtKB:Q8IZA3",
  "gene_name": "Histone H1.8",
  "gene_symbol": "H1-8",
  "term_id": "GO:0031492",
  "term_label": "nucleosomal DNA binding"
}